momilactone-A synthase [NAD(P)H] activity [GO:0102960] (molecular function) Definition: Catalysis of the reaction: 3beta-hydroxy-9beta-pimara-7,15-diene-19,6beta-olide + NAD(P) = momilactone A + H+ + NAD(P)H. Sources: EC:1.1.1.295 Relationships: is a type of oxidoreductase activity, acting on the CH-OH group of donors, NAD or NADP as acceptor [GO:0016616]